{
  "term_id": "UNKNOWN:0003",
  "gene_symbol": "TSSK4",
  "gene_name": "Testis-specific serine_threonine-protein kinase 4",
  "term_label": "Unknown cellular component",
  "gene": "UniProtKB:Q6SA08"
}